{
  "term_label": "olfactory receptor activity",
  "gene_symbol": "OR6A2",
  "gene_name": "Olfactory receptor 6A2",
  "term_id": "GO:0004984",
  "gene": "UniProtKB:O95222"
}